{
  "gene_symbol": "TGFBR2",
  "gene": "UniProtKB:P37173",
  "term_id": "GO:0016361",
  "term_label": "activin receptor activity, type I",
  "gene_name": "TGF-beta receptor type-2"
}